DNA nuclease activity [GO:0004536] (molecular function) Definition: Catalysis of the cleavage of ester linkages within deoxyribonucleic acid. Relationships: is_a nuclease activity [GO:0004518]; is a type of catalytic activity, acting on DNA [GO:0140097]; is part of DNA metabolic process [GO:0006259] Also known as: deoxyribonuclease activity, caspase-activated deoxyribonuclease activity Subtypes: DNA endonuclease activity [GO:0004520], DNA exonuclease activity [GO:0004529] Regulation: positively regulated by positive regulation of deoxyribonuclease activity [GO:0032077]; negatively regulated by deoxyribonuclease inhibitor activity [GO:0060703] Sources: GOC:mah, ISBN:0198547684